glycolytic process through glucose-1-phosphate [GO:0061622] (biological process) Relationships: is a type of glycolytic process through glucose-6-phosphate [GO:0061620]; has part GO:0004614 Subtypes: glycolytic process from galactose [GO:0061623], glycolysis from storage polysaccharide through glucose-1-phosphate [GO:0093001] Sources: GOC:dph, ISBN:0201090910 Definition: The chemical reactions and pathways through a glucose-1-phosphate intermediate that result in the catabolism of a carbohydrate into pyruvate, with the concomitant production of a small amount of ATP.